cellular response to pyrimidine ribonucleotide [GO:1905835] (biological process) Relationships: is a type of cellular response to nitrogen compound [GO:1901699]; is a type of cellular response to oxygen-containing compound [GO:1901701]; is a type of response to pyrimidine ribonucleotide [GO:1905834] Definition: Any process that results in a change in state or activity of a cell (in terms of movement, secretion, enzyme production, gene expression, etc.) as a result of a pyrimidine ribonucleotide stimulus. References: PMID:22065602 Sources: GOC:TermGenie, GO_REF:0000071